FERRY complex [GO:0160271] (cellular component) Definition: A protein complex that directly interacts with mRNAs and Rab5, functions as a Rab5 effector, recruits mRNAs and ribosomes to early endosomes through direct mRNA-interaction, is composed of five subunits, TBCK, PPP1R21, FERRY3, CRYZL1 and GATD1 with a ratio of 1:2:1:2:4, respectively. Relationships: is a type of protein-containing complex [GO:0032991] References: PMID:37267905, PMID:37267906 Also known as: FERRY RAB5 effector complex, five-subunit endosomal Rab5 complex, RNA/ribosome intermediary complex